{
  "term_id": "GO:0005886",
  "gene": "UniProtKB:Q16206",
  "gene_name": "Ecto-NOX disulfide-thiol exchanger 2",
  "gene_symbol": "ENOX2",
  "term_label": "plasma membrane"
}